cholinergic synapse [GO:0098981] (cellular component) Definition: A synapse that uses acetylcholine as a neurotransmitter. Sources: GOC:dos Relationships: is a type of GO:0045202 Subtypes: neuromuscular junction of skeletal muscle fiber [GO:0098522]